{
  "gene": "UniProtKB:Q9NRD5",
  "gene_symbol": "PICK1",
  "term_id": "GO:0032588",
  "term_label": "trans-Golgi network membrane",
  "gene_name": "PRKCA-binding protein"
}